{
  "gene": "UniProtKB:Q7Z3Y7",
  "gene_symbol": "KRT28",
  "term_id": "GO:0031069",
  "term_label": "hair follicle morphogenesis",
  "gene_name": "Keratin, type I cytoskeletal 28"
}